sulfide oxidation [GO:0019418] (biological process) Definition: The chemical reactions and pathways resulting in the conversion of sulfide to elemental sulfur in a higher oxidation state, or to sulfite or sulfate. Sources: MetaCyc:Sulfide-Oxidation Also known as: sulphide oxidation Subtypes: sulfide oxidation, using sulfide:quinone oxidoreductase [GO:0070221], sulfide oxidation, using sulfide dehydrogenase [GO:0070222], sulfide oxidation, using sulfur dioxygenase [GO:0070223] Relationships: is a type of sulfur compound metabolic process [GO:0006790]